{
  "gene_name": "Uromodulin-like 1",
  "gene": "UniProtKB:Q5DID0",
  "term_label": "Unknown biological process",
  "gene_symbol": "UMODL1",
  "term_id": "UNKNOWN:0002"
}